{
  "term_label": "positive regulation of axon regeneration",
  "gene": "UniProtKB:P26441",
  "gene_symbol": "CNTF",
  "gene_name": "Ciliary neurotrophic factor",
  "term_id": "GO:0048680"
}